oxidoreductase activity, acting on metal ions, oxygen as acceptor [GO:0016724] (molecular function) Also known as: oxidoreductase activity, oxidizing metal ions, oxygen as acceptor Subtypes: ferroxidase activity [GO:0004322] Relationships: is a type of oxidoreductase activity, acting on metal ions [GO:0016722] Sources: GOC:mah Definition: Catalysis of an oxidation-reduction in which the oxidation state of metal ion is altered and oxygen acts as an electron acceptor.